ammelide aminohydrolase activity [GO:0018754] (molecular function) Definition: Catalysis of the reaction: ammelide + H2O = cyanuric acid + NH3. References: PMID:1991731 Relationships: is a type of hydrolase activity, acting on carbon-nitrogen (but not peptide) bonds, in linear amidines [GO:0016813]